S-methylmethionine metabolic process [GO:0033477] (biological process) References: PMID:12692340 Sources: GOC:mah Also known as: S-methylmethionine metabolism Definition: The chemical reactions and pathways involving S-methyl-methionine (SMM). SMM can be converted to methionine by donating a methyl group to homocysteine, and concurrent operation of this reaction and that mediated by MMT sets up the SMM cycle. Subtypes: S-methylmethionine biosynthetic process [GO:0010250], S-methylmethionine cycle [GO:0033528] Relationships: is a type of GO:0006575; is a type of sulfur compound metabolic process [GO:0006790]